{
  "gene_symbol": "VPS13A",
  "term_id": "GO:0006914",
  "term_label": "autophagy",
  "gene": "UniProtKB:Q96RL7",
  "gene_name": "Intermembrane lipid transfer protein VPS13A"
}